{
  "term_id": "GO:0045944",
  "gene_name": "CREB-regulated transcription coactivator 3",
  "gene_symbol": "CRTC3",
  "gene": "UniProtKB:Q6UUV7",
  "term_label": "positive regulation of transcription by RNA polymerase II"
}